{
  "gene_name": "Histone H2B type 1-K",
  "term_label": "nucleus",
  "gene_symbol": "H2BC12",
  "gene": "UniProtKB:O60814",
  "term_id": "GO:0005634"
}